{
  "gene_name": "SCY1-like protein 2",
  "gene_symbol": "SCYL2",
  "term_id": "UNKNOWN:0003",
  "term_label": "Unknown cellular component",
  "gene": "UniProtKB:Q6P3W7"
}